{
  "gene_symbol": "GABRA3",
  "gene": "UniProtKB:P34903",
  "gene_name": "Gamma-aminobutyric acid receptor subunit alpha-3",
  "term_id": "GO:1902476",
  "term_label": "chloride transmembrane transport"
}